3-ketosteroid 9-alpha-monooxygenase activity [GO:0036200] (molecular function) Definition: Catalysis of the reaction: androsta-1,4-diene-3,17-dione + 2 H+ + O2 + 2 reduced [2Fe-2S]-[ferredoxin] = 9alpha-hydroxyandrosta-1,4-diene-3,17-dione + H2O + 2 oxidized [2Fe-2S]-[ferredoxin]. Sources: EC:1.14.15.30 Also known as: 3-ketosteroid 9alpha-hydroxylase activity, KshAB activity Relationships: is a type of oxidoreductase activity, acting on paired donors, with incorporation or reduction of molecular oxygen, reduced iron-sulfur protein as one donor, and incorporation of one atom of oxygen [GO:0016713]